{
  "gene": "UniProtKB:Q9Y2V2",
  "term_id": "GO:0043488",
  "gene_symbol": "CARHSP1",
  "term_label": "regulation of mRNA stability",
  "gene_name": "Calcium-regulated heat-stable protein 1"
}